F bouton [GO:1990025] (cellular component) Relationships: is a type of terminal bouton [GO:0043195] Definition: Synaptic bouton found in the ventral horn of the spinal cord. F boutons range in diameter from 0.5 to 7 um and contain flattened or pleomorphic synaptic vesicles. Sources: NIF_Subcellular:nlx_subcell_100206